{
  "term_id": "GO:0008432",
  "gene_name": "C-Jun-amino-terminal kinase-interacting protein 2",
  "gene_symbol": "MAPK8IP2",
  "term_label": "JUN kinase binding",
  "gene": "UniProtKB:Q13387"
}